{
  "term_id": "GO:0005634",
  "gene_name": "Transcription factor HES-2",
  "gene": "UniProtKB:Q9Y543",
  "gene_symbol": "HES2",
  "term_label": "nucleus"
}